convergent extension involved in imaginal disc-derived wing morphogenesis [GO:0090253] (biological process) Definition: The morphogenetic process in which the wing epithelium narrows along one axis and lengthens in a perpendicular axis that contributes to imaginal disc-derived wing morphogenesis. Relationships: is a type of GO:0009886; is a type of convergent extension involved in organogenesis [GO:0060029]; is part of imaginal disc-derived wing morphogenesis [GO:0007476] Sources: GOC:ascb_2009, GOC:dph, GOC:tb